{
  "term_id": "UNKNOWN:0003",
  "term_label": "Unknown cellular component",
  "gene_name": "Ankyrin repeat domain-containing protein 40",
  "gene": "UniProtKB:Q6AI12",
  "gene_symbol": "ANKRD40"
}